{
  "term_id": "GO:0006357",
  "gene_name": "Zinc finger protein 776",
  "gene_symbol": "ZNF776",
  "term_label": "regulation of transcription by RNA polymerase II",
  "gene": "UniProtKB:Q68DI1"
}